dextrin catabolic process [GO:1901027] (BP) Relationships: is a type of GO:0009251 Subtypes: cellodextrin catabolic process [GO:2000890], cyclodextrin catabolic process [GO:2000901] Also known as: dextrin breakdown, dextrin catabolism, dextrin degradation Sources: GOC:TermGenie Definition: The chemical reactions and pathways resulting in the breakdown of dextrin.